{
  "term_id": "UNKNOWN:0002",
  "term_label": "Unknown biological process",
  "gene_symbol": "BCL2L13",
  "gene": "UniProtKB:Q9BXK5",
  "gene_name": "Bcl-2-like protein 13"
}